{
  "term_label": "proteasome binding",
  "gene_name": "Proteasome assembly chaperone 1",
  "gene_symbol": "PSMG1",
  "term_id": "GO:0070628",
  "gene": "UniProtKB:O95456"
}